cysteine-type peptidase activity [GO:0008234] (MF) Sources: GOC:mah, https://www.ebi.ac.uk/merops/about/glossary.shtml#CATTYPE Subtypes: cysteine-type endopeptidase activity [GO:0004197], cysteine-type deubiquitinase activity [GO:0004843], pyroglutamyl-peptidase activity [GO:0016920], deSUMOylase activity [GO:0016929], ISG15-specific peptidase activity [GO:0019785], GO:0034722, cysteine-type exopeptidase activity [GO:0070004], GO:0071567, cysteine-type deNEDDylase activity [GO:0140757] Relationships: is_a GO:0008233 Also known as: cysteine protease activity, thiol protease activity Definition: Catalysis of the hydrolysis of peptide bonds in a polypeptide chain by a mechanism in which the sulfhydryl group of a cysteine residue at the active center acts as a nucleophile.